{
  "gene": "UniProtKB:Q9UJW8",
  "term_id": "GO:0000977",
  "term_label": "RNA polymerase II transcription regulatory region sequence-specific DNA binding",
  "gene_symbol": "ZNF180",
  "gene_name": "Zinc finger protein 180"
}